cellular response to nonane [GO:1902781] (biological process) Definition: Any process that results in a change in state or activity of a cell (in terms of movement, secretion, enzyme production, gene expression, etc.) as a result of a nonane stimulus. Relationships: is a type of GO:1902779; is a type of response to nonane [GO:1902780] References: PMID:22958739 Sources: GOC:TermGenie, GOC:mengo_curators, GO_REF:0000071